{
  "term_label": "sodium channel regulator activity",
  "gene": "UniProtKB:O00168",
  "gene_symbol": "FXYD1",
  "gene_name": "Phospholemman",
  "term_id": "GO:0017080"
}